{
  "gene_symbol": "IGLV3-12",
  "term_label": "immunoglobulin complex",
  "gene_name": "Immunoglobulin lambda variable 3-12",
  "term_id": "GO:0019814",
  "gene": "UniProtKB:A0A075B6K2"
}